{
  "gene_name": "Bardet-Biedl syndrome 2 protein",
  "gene_symbol": "BBS2",
  "term_id": "GO:0036064",
  "gene": "UniProtKB:Q9BXC9",
  "term_label": "ciliary basal body"
}